{
  "gene_symbol": "TPSAB1",
  "term_label": "extracellular space",
  "gene": "UniProtKB:Q15661",
  "gene_name": "Tryptase alpha_beta-1",
  "term_id": "GO:0005615"
}